{
  "gene": "UniProtKB:Q9NZT2",
  "gene_symbol": "OGFR",
  "term_id": "UNKNOWN:0002",
  "gene_name": "Opioid growth factor receptor",
  "term_label": "Unknown biological process"
}